{
  "term_label": "plasma membrane tubulation",
  "term_id": "GO:0097320",
  "gene_name": "Protein kinase C and casein kinase substrate in neurons protein 2",
  "gene": "UniProtKB:Q9UNF0",
  "gene_symbol": "PACSIN2"
}